{
  "term_id": "GO:0005739",
  "term_label": "mitochondrion",
  "gene_name": "Thiosulfate sulfurtransferase",
  "gene": "UniProtKB:Q16762",
  "gene_symbol": "TST"
}